{
  "term_id": "GO:1902476",
  "gene_name": "Chloride anion exchanger",
  "gene": "UniProtKB:P40879",
  "gene_symbol": "SLC26A3",
  "term_label": "chloride transmembrane transport"
}